{
  "gene_name": "Sodium-dependent serotonin transporter",
  "term_id": "GO:0006865",
  "term_label": "amino acid transport",
  "gene": "UniProtKB:P31645",
  "gene_symbol": "SLC6A4"
}